{
  "gene_name": "N-acetyllactosaminide beta-1,3-N-acetylglucosaminyltransferase 4",
  "gene": "UniProtKB:Q9C0J1",
  "term_id": "GO:0030311",
  "term_label": "poly-N-acetyllactosamine biosynthetic process",
  "gene_symbol": "B3GNT4"
}